telium development [GO:0075275] (biological process) Definition: The process that leads to the development of a telium, which is a teliospore-bearing sorus of the rust fungi. Sources: GOC:pamgo_curators Relationships: is a type of spore-bearing structure development [GO:0075259] Regulation: regulated by GO:0075276; positively regulated by GO:0075277; negatively regulated by GO:0075278